stem cell population maintenance [GO:0019827] (BP) Sources: GOC:mah, ISBN:0878932437 Relationships: is a type of multicellular organismal process [GO:0032501]; is a type of GO:0098727 Subtypes: maintenance of meristem identity [GO:0010074], germ-line stem cell population maintenance [GO:0030718], GO:0035019, GO:0097150 Also known as: maintenance of pluripotency Definition: The process by which an organism or tissue maintains a population of stem cells of a single type. This can be achieved by a number of mechanisms: stem cell asymmetric division maintains stem cell numbers; stem cell symmetric division increases them; maintenance of a stem cell niche maintains the conditions for commitment to the stem cell fate for some types of stem cell; stem cells may arise de novo from other cell types. Regulation: negatively regulated by GO:1902455; positively regulated by positive regulation of stem cell population maintenance [GO:1902459]; regulated by regulation of stem cell population maintenance [GO:2000036]